{
  "term_label": "nuclear-transcribed mRNA catabolic process, 3'-5' exonucleolytic nonsense-mediated decay",
  "gene": "UniProtKB:Q15477",
  "gene_symbol": "SKIC2",
  "term_id": "GO:0070478",
  "gene_name": "Superkiller complex protein 2"
}